{
  "term_label": "proteasome binding",
  "gene_symbol": "ADRM1",
  "gene": "UniProtKB:Q16186",
  "term_id": "GO:0070628",
  "gene_name": "Proteasomal ubiquitin receptor ADRM1"
}